5-aminolevulinic acid import across plasma membrane [GO:0140484] (biological process) References: PMID:31989647 Relationships: is a type of organic cation transport [GO:0015695]; is a type of monocarboxylic acid transport [GO:0015718]; is a type of nitrogen compound transport [GO:0071705]; is a type of GO:0089718; is a type of GO:1905039 Definition: The directed movement of 5-aminolevulinic acid from outside of a cell, across the plasma membrane and into the cytosol.